inner cell mass cell differentiation [GO:0001826] (biological process) Note: See also the Anatomical Dictionary for Mouse Development ontology terms 'TS4, inner cell mass ; EMAP:14'. Relationships: is a type of GO:0030154; BFO_0000050 blastocyst formation [GO:0001825] Sources: GOC:dph, ISBN:0124020607, ISBN:0198542771 Definition: The process in which a relatively unspecialized cell acquires specialized features of an inner cell mass cell.